mitotic DNA replication initiation [GO:1902975] (biological process) Sources: GOC:TermGenie, GO_REF:0000060 Definition: Any DNA replication initiation involved in mitotic cell cycle DNA replication. Regulation: regulated by GO:1903466; negatively regulated by negative regulation of mitotic DNA replication initiation [GO:1903467]; positively regulated by positive regulation of DNA replication initiation [GO:1903468] Also known as: DNA replication initiation involved in mitotic cell cycle DNA replication Relationships: is a type of nuclear cell cycle DNA replication initiation [GO:1902315]; is a type of mitotic cell cycle process [GO:1903047]; is part of mitotic DNA replication [GO:1902969]